pyrimidine ribonucleoside biosynthetic process [GO:0046132] (BP) Definition: The chemical reactions and pathways resulting in the formation of any ribonucleoside, a nucleoside in which a pyrimidine base is linked to a ribose (beta-D-ribofuranose) molecule. Relationships: is_a ribonucleoside biosynthetic process [GO:0042455]; is a type of pyrimidine ribonucleoside metabolic process [GO:0046131]; is a type of pyrimidine nucleoside biosynthetic process [GO:0046134] Sources: GOC:ai Subtypes: uridine biosynthetic process [GO:0046109] Also known as: pyrimidine ribonucleoside anabolism, pyrimidine ribonucleoside biosynthesis, pyrimidine ribonucleoside formation, pyrimidine ribonucleoside synthesis